{
  "gene": "UniProtKB:Q9NVN8",
  "gene_name": "Guanine nucleotide-binding protein-like 3-like protein",
  "term_label": "Unknown biological process",
  "gene_symbol": "GNL3L",
  "term_id": "UNKNOWN:0002"
}